{
  "gene_name": "Zinc finger protein 629",
  "term_id": "GO:0006357",
  "gene_symbol": "ZNF629",
  "gene": "UniProtKB:Q9UEG4",
  "term_label": "regulation of transcription by RNA polymerase II"
}